{
  "gene_name": "Protein orai-2",
  "term_label": "membrane",
  "term_id": "GO:0016020",
  "gene_symbol": "ORAI2",
  "gene": "UniProtKB:Q96SN7"
}